{
  "term_id": "GO:0045595",
  "gene_symbol": "RUNX2",
  "term_label": "regulation of cell differentiation",
  "gene": "UniProtKB:Q13950",
  "gene_name": "Runt-related transcription factor 2"
}